cellular response to monoamine stimulus [GO:0071868] (biological process) Definition: Any process that results in a change in state or activity of a cell (in terms of movement, secretion, enzyme production, gene expression, etc.) as a result of a monoamine stimulus. A monoamine is any of a group of molecular messengers that contain one amino group that is connected to an aromatic ring by ethylene group (-CH2-CH2-). Monoamines are derived from the aromatic amino acids phenylalanine, tyrosine, histidine and tryptophan. Sources: GOC:mah Relationships: is a type of GO:0071867; is a type of cellular response to nitrogen compound [GO:1901699] Subtypes: cellular response to catecholamine stimulus [GO:0071870], cellular response to serotonin [GO:1904015]